{
  "gene": "UniProtKB:Q8IZF3",
  "gene_symbol": "ADGRF4",
  "term_label": "G protein-coupled receptor activity",
  "term_id": "GO:0004930",
  "gene_name": "Adhesion G protein-coupled receptor F4"
}